{
  "term_label": "Golgi apparatus",
  "gene": "UniProtKB:Q8TEB7",
  "gene_name": "E3 ubiquitin-protein ligase RNF128",
  "gene_symbol": "RNF128",
  "term_id": "GO:0005794"
}